{
  "gene": "UniProtKB:O43365",
  "gene_symbol": "HOXA3",
  "gene_name": "Homeobox protein Hox-A3",
  "term_id": "GO:0000981",
  "term_label": "DNA-binding transcription factor activity, RNA polymerase II-specific"
}